cerebellar cortex morphogenesis [GO:0021696] (biological process) Sources: GOC:cls, GOC:dgh, GOC:dph, GOC:jid, GO_REF:0000021 Relationships: is a type of anatomical structure morphogenesis [GO:0009653]; BFO_0000050 GO:0021587; is part of cerebellar cortex development [GO:0021695] Definition: The process in which the anatomical structure of the cranial nerves are generated and organized. The cerebellar cortex is a thin mantle of gray matter that covers the surface of each cerebral hemisphere. It has a characteristic morphology with convolutions (gyri) and crevices (sulci) that have specific functions. Six layers of nerve cells and the nerve pathways that connect them comprise the cerebellar cortex. Together, these regions are responsible for the processes of conscious thought, perception, emotion and memory as well as advanced motor function.